{
  "gene": "UniProtKB:Q01415",
  "term_label": "galactokinase activity",
  "term_id": "GO:0004335",
  "gene_name": "N-acetylgalactosamine kinase",
  "gene_symbol": "GALK2"
}